ionotropic taste receptor activity [GO:0170021] (molecular function) Definition: Enables the transmembrane transfer of an ion by a channel that opens when a soluble compound has been bound by the channel complex or one of its constituent parts. References: PMID:36828965 Subtypes: ionotropic salty taste receptor activity [GO:0033039], ionotropic bitter taste receptor activity [GO:0170022], GO:0170023 Relationships: is a type of taste receptor activity [GO:0008527]; is a type of GO:0015276